{
  "gene_symbol": "GOLM2",
  "term_id": "UNKNOWN:0002",
  "gene_name": "Protein GOLM2",
  "term_label": "Unknown biological process",
  "gene": "UniProtKB:Q6P4E1"
}